{
  "gene_symbol": "IGHV3-13",
  "term_id": "GO:0016064",
  "gene": "UniProtKB:P01766",
  "gene_name": "Immunoglobulin heavy variable 3-13",
  "term_label": "immunoglobulin mediated immune response"
}